{
  "gene_name": "Putative ubiquitin carboxyl-terminal hydrolase 41",
  "term_label": "Unknown biological process",
  "gene_symbol": "USP41",
  "term_id": "UNKNOWN:0002",
  "gene": "UniProtKB:Q3LFD5"
}